{
  "term_label": "Unknown cellular component",
  "gene_name": "Transmembrane protein 89",
  "term_id": "UNKNOWN:0003",
  "gene_symbol": "TMEM89",
  "gene": "UniProtKB:A2RUT3"
}